{
  "gene_symbol": "ZNF860",
  "term_id": "GO:0006357",
  "gene_name": "Zinc finger protein 860",
  "term_label": "regulation of transcription by RNA polymerase II",
  "gene": "UniProtKB:A6NHJ4"
}